{
  "gene_name": "Aldehyde dehydrogenase 1A1",
  "term_label": "cytosol",
  "term_id": "GO:0005829",
  "gene": "UniProtKB:P00352",
  "gene_symbol": "ALDH1A1"
}